{
  "gene_name": "Mitogen-activated protein kinase 14",
  "gene": "UniProtKB:Q16539",
  "term_id": "GO:0004674",
  "term_label": "protein serine/threonine kinase activity",
  "gene_symbol": "MAPK14"
}